{
  "gene": "UniProtKB:Q9NR61",
  "gene_symbol": "DLL4",
  "term_id": "GO:0045746",
  "gene_name": "Delta-like protein 4",
  "term_label": "negative regulation of Notch signaling pathway"
}